{
  "term_label": "plasma membrane",
  "gene_symbol": "GPR17",
  "term_id": "GO:0005886",
  "gene": "UniProtKB:Q13304",
  "gene_name": "Uracil nucleotide_cysteinyl leukotriene receptor"
}